regulation of DNA-binding transcription factor activity [GO:0051090] (biological process) Definition: Any process that modulates the frequency, rate or extent of the activity of a transcription factor, any factor involved in the initiation or regulation of transcription. Sources: GOC:ai Also known as: regulation of transcription factor activity, regulation of DNA binding transcription factor activity, regulation of sequence-specific DNA binding transcription factor activity, regulation of androgen receptor activity, regulation of thyroid hormone receptor activity Subtypes: negative regulation of DNA-binding transcription factor activity [GO:0043433], positive regulation of DNA-binding transcription factor activity [GO:0051091], negative regulation of hh target transcription factor activity [GO:1990787] Relationships: is a type of GO:0006355; is a type of regulation of molecular function [GO:0065009]; regulates DNA-binding transcription factor activity [GO:0003700]